MutSbeta complex binding [GO:0032408] (molecular function) Definition: Binding to a MutSbeta mismatch repair complex. Sources: GOC:vk Relationships: is a type of mismatch repair complex binding [GO:0032404]